{
  "term_id": "GO:0005730",
  "gene": "UniProtKB:Q86WX3",
  "gene_symbol": "RPS19BP1",
  "term_label": "nucleolus",
  "gene_name": "Active regulator of SIRT1"
}